{
  "term_label": "secretory granule",
  "term_id": "GO:0030141",
  "gene_name": "Syntaxin-binding protein 1",
  "gene": "UniProtKB:P61764",
  "gene_symbol": "STXBP1"
}